{
  "term_id": "GO:0005634",
  "term_label": "nucleus",
  "gene_name": "Nuclear factor 1 A-type",
  "gene_symbol": "NFIA",
  "gene": "UniProtKB:Q12857"
}